{
  "gene_name": "Tumor necrosis factor receptor superfamily member 6",
  "term_label": "CD95 death-inducing signaling complex",
  "gene_symbol": "FAS",
  "gene": "UniProtKB:P25445",
  "term_id": "GO:0031265"
}